{
  "term_label": "Unknown cellular component",
  "gene": "UniProtKB:O60315",
  "term_id": "UNKNOWN:0003",
  "gene_symbol": "ZEB2",
  "gene_name": "Zinc finger E-box-binding homeobox 2"
}